{
  "term_label": "ciliary transition fiber",
  "gene": "UniProtKB:Q9Y592",
  "gene_symbol": "CEP83",
  "gene_name": "Centrosomal protein of 83 kDa",
  "term_id": "GO:0097539"
}